{
  "gene_name": "Ubiquitin domain-containing protein 2",
  "term_label": "Unknown cellular component",
  "gene": "UniProtKB:Q8WUN7",
  "gene_symbol": "UBTD2",
  "term_id": "UNKNOWN:0003"
}